synaptic receptor adaptor activity [GO:0030160] (molecular function) Definition: The binding activity of a molecule that provides a physical support bridging a synaptic signaling receptor and a downstream signaling molecule. Relationships: is a type of signaling receptor complex adaptor activity [GO:0030159] Also known as: GKAP/Homer scaffold activity, GKAP/Homer scaffold protein, postsynaptic density scaffold protein References: PMID:10506216